positive regulation of neural crest formation [GO:0090300] (biological process) Subtypes: positive regulation of neural crest cell fate specification [GO:1905297] Definition: Any process that increases the rate, frequency, or extent of neural crest formation. Neural crest formation is the formation of the specialized region of ectoderm between the neural ectoderm (neural plate) and non-neural ectoderm. The neural crest gives rise to the neural crest cells that migrate away from this region as neural tube formation proceeds. Sources: GOC:tb Relationships: is a type of positive regulation of epithelial to mesenchymal transition [GO:0010718]; is a type of regulation of neural crest formation [GO:0090299]; positively regulates neural crest formation [GO:0014029]